{
  "gene": "UniProtKB:Q6PCB7",
  "term_id": "GO:0001579",
  "gene_name": "Long-chain fatty acid transport protein 1",
  "gene_symbol": "SLC27A1",
  "term_label": "medium-chain fatty acid transport"
}